regulation of pro-B cell differentiation [GO:2000973] (biological process) Sources: GOC:obol Also known as: regulation of pro-B lymphocyte differentiation, regulation of pro-B cell development Subtypes: GO:2000974, positive regulation of pro-B cell differentiation [GO:2000975] Relationships: is a type of regulation of lymphoid progenitor cell differentiation [GO:1905456]; regulates pro-B cell differentiation [GO:0002328] Definition: Any process that modulates the frequency, rate or extent of pro-B cell differentiation.